{
  "term_id": "GO:0005868",
  "gene_name": "Dynein light chain roadblock-type 2",
  "term_label": "cytoplasmic dynein complex",
  "gene": "UniProtKB:Q8TF09",
  "gene_symbol": "DYNLRB2"
}